nucleoside deoxyribosyltransferase activity [GO:0050144] (molecular function) Relationships: is a type of pentosyltransferase activity [GO:0016763] Sources: EC:2.4.2.6, MetaCyc:NUCLEOSIDE-DEOXYRIBOSYLTRANSFERASE-RXN Definition: Catalysis of the reaction: 2-deoxy-D-ribosyl-base1 + base2 = 2-deoxy-D-ribosyl-base2 + base1. Also known as: deoxyribose transferase activity, nucleoside deoxyribosyltransferase I (purine nucleoside:purine deoxyribosyltransferase: strictly specific for transfer between purine bases), nucleoside deoxyribosyltransferase II [purine(pyrimidine) nucleoside:purine(pyrimidine) deoxyribosyltransferase], nucleoside trans-N-deoxyribosylase activity, nucleoside:purine(pyrimidine) deoxy-D-ribosyltransferase activity, purine(pyrimidine) nucleoside:purine(pyrimidine) deoxyribosyl transferase activity, trans-N-deoxyribosylase activity, trans-N-glycosidase activity, trans-deoxyribosylase activity